{
  "gene_name": "Ewing's tumor-associated antigen 1",
  "term_label": "replication fork processing",
  "term_id": "GO:0031297",
  "gene": "UniProtKB:Q9NY74",
  "gene_symbol": "ETAA1"
}